{
  "term_id": "GO:0004857",
  "gene_name": "UDP-glucuronosyltransferase 1A9",
  "gene": "UniProtKB:O60656",
  "term_label": "enzyme inhibitor activity",
  "gene_symbol": "UGT1A9"
}